{
  "gene_name": "SUN domain-containing protein 2",
  "term_id": "GO:0005635",
  "gene_symbol": "SUN2",
  "gene": "UniProtKB:Q9UH99",
  "term_label": "nuclear envelope"
}